{
  "term_id": "GO:1902017",
  "gene": "UniProtKB:Q8NF91",
  "gene_symbol": "SYNE1",
  "gene_name": "Nesprin-1",
  "term_label": "regulation of cilium assembly"
}